anaerobic pectin catabolic process [GO:1990489] (biological process) Definition: The chemical reactions and pathways resulting in the breakdown of pectin, a polymer containing a backbone of alpha-1,4-linked D-galacturonic acid residues, in the absence of oxygen. References: PMID:23079077 Sources: GOC:mengo_curators Also known as: anaerobic pectin degradation Relationships: is a type of pectin catabolic process [GO:0045490]